{
  "gene_symbol": "SRF",
  "term_label": "serum response element binding",
  "gene_name": "Serum response factor",
  "term_id": "GO:0010736",
  "gene": "UniProtKB:P11831"
}